{
  "gene": "UniProtKB:O95466",
  "term_label": "cortical actin cytoskeleton organization",
  "gene_symbol": "FMNL1",
  "gene_name": "Formin-like protein 1",
  "term_id": "GO:0030866"
}